{
  "gene_name": "Putative tyrosine-protein phosphatase TPTE",
  "term_label": "cytosol",
  "term_id": "GO:0005829",
  "gene_symbol": "TPTE",
  "gene": "UniProtKB:P56180"
}